{
  "term_label": "RNA polymerase II CTD heptapeptide repeat phosphatase activity",
  "term_id": "GO:0008420",
  "gene_name": "RNA polymerase II subunit A C-terminal domain phosphatase SSU72 like protein 3",
  "gene": "UniProtKB:A0A1W2PQJ5",
  "gene_symbol": "SSU72L3"
}